L-cysteate sulfo-lyase activity [GO:0034011] (molecular function) Sources: EC:4.4.1.25, RHEA:13441 Relationships: is a type of carbon-sulfur lyase activity [GO:0016846] Definition: Catalysis of the reaction: L-cysteate + H2O = NH4 + pyruvate + sulfite. Also known as: CuyA, L-cysteate bisulfite-lyase (deaminating; pyruvate-forming) activity, L-cysteate sulfo-lyase (deaminating) activity